{
  "term_id": "GO:0046330",
  "gene": "UniProtKB:Q9NRW4",
  "term_label": "positive regulation of JNK cascade",
  "gene_symbol": "DUSP22",
  "gene_name": "Dual specificity protein phosphatase 22"
}